{
  "gene_symbol": "ANKS1B",
  "term_id": "GO:0099523",
  "gene": "UniProtKB:Q7Z6G8",
  "gene_name": "Ankyrin repeat and sterile alpha motif domain-containing protein 1B",
  "term_label": "presynaptic cytosol"
}